{
  "term_id": "GO:0070523",
  "term_label": "11-beta-hydroxysteroid dehydrogenase (NAD+) activity",
  "gene_symbol": "HSD11B2",
  "gene": "UniProtKB:P80365",
  "gene_name": "11-beta-hydroxysteroid dehydrogenase type 2"
}